pre-mRNA branch point binding [GO:0045131] (molecular function) Definition: Binding to a pre-mRNA branch point sequence, located upstream of the 3' splice site. References: PMID:11691992, PMID:9722632 Relationships: is a type of pre-mRNA binding [GO:0036002]